positive regulation of metallopeptidase activity [GO:1905050] (biological process) Subtypes: positive regulation of metalloendopeptidase activity [GO:1904685] Also known as: up regulation of metallopeptidase activity, up-regulation of metallopeptidase activity, upregulation of metallopeptidase activity, activation of metallopeptidase activity, activation of metalloprotease activity, activation of metalloproteinase activity, positive regulation of metalloprotease activity, positive regulation of metalloproteinase activity, up regulation of metalloprotease activity, up regulation of metalloproteinase activity, up-regulation of metalloprotease activity, up-regulation of metalloproteinase activity, upregulation of metalloprotease activity, upregulation of metalloproteinase activity References: PMID:26473732 Sources: GOC:TermGenie, GO_REF:0000059 Relationships: is a type of GO:0010952; is a type of regulation of metallopeptidase activity [GO:1905048]; positively regulates metallopeptidase activity [GO:0008237] Definition: Any process that activates or increases the frequency, rate or extent of metallopeptidase activity.